{
  "term_id": "GO:0005085",
  "gene_name": "PH and SEC7 domain-containing protein 4",
  "gene_symbol": "PSD4",
  "gene": "UniProtKB:Q8NDX1",
  "term_label": "guanyl-nucleotide exchange factor activity"
}